{
  "term_id": "GO:0005544",
  "term_label": "calcium-dependent phospholipid binding",
  "gene_name": "Cytosolic phospholipase A2 beta",
  "gene_symbol": "PLA2G4B",
  "gene": "UniProtKB:P0C869"
}